{
  "term_id": "GO:0030276",
  "gene_symbol": "AP2B1",
  "gene_name": "AP-2 complex subunit beta",
  "gene": "UniProtKB:P63010",
  "term_label": "clathrin binding"
}